steviol 13-O glucosyltransferase activity [GO:0102377] (molecular function) Sources: RHEA:61732 Definition: Catalysis of the reaction: steviol + UDP-alpha-D-glucose = H+ + steviolmonoside + UDP. Relationships: is_a GO:0016758